Fc-alpha receptor I complex [GO:0032999] (cellular component) Definition: A protein complex composed of an Fc-alpha R alpha chain and an Fc-epsilon RI gamma chain dimer with or without additional signaling components. The complex functions primarily as an activating receptor for IgA. References: PMID:12524384 Sources: GOC:add, ISBN:0781735149 Relationships: is a type of Fc receptor complex [GO:0032997] Also known as: IgA receptor complex, immunoglobulin A receptor complex, FcaRI complex